platelet-derived growth factor receptor-ligand complex [GO:1990270] (cellular component) Relationships: is a type of plasma membrane protein complex [GO:0098797]; has part receptor complex [GO:0043235]; has part platelet-derived growth factor complex [GO:1990265] Note: An example of this is PDGFA-PGFRA in human (UniProt symbols P04085, P16234) in PMID:7679113 (inferred from direct assay). Also known as: PDGF complex, receptor-ligand complex, PDGF receptor-ligand complex, PDGF-AA-receptor alpha complex, PDGF-AB-receptor alpha complex, PDGF-AB-receptor beta complex, PDGF-BB-receptor alpha complex, PDGF-BB-receptor alpha-beta complex, PDGF-BB-receptor beta complex, PDGF-CC-receptor alpha complex, PDGF-CC-receptor alpha-beta complex, PDGF-CC-receptor beta complex, PDGF-DD-receptor alpha-beta complex, PDGF-DD-receptor beta complex Definition: A tetrameric protein complex consisting of two platelet-derived growth factor (PDGF) receptor subunits and two PDGF ligand subunits. Binding of the PDGF ligand dimer to the PDGF receptor in the plasma membrane induces receptor dimerization and activation. PDGFs are involved in a wide variety of signaling processes and are found in all vertebrates. At least two different receptor chains (A and B) and four types of ligand chains (A, B, C, and D) are known forming a wide variety of combinations of receptor-ligand complexes. References: PMID:11331882 Sources: GOC:bhm